alcohol sulfotransferase activity [GO:0004027] (molecular function) Definition: Catalysis of the reaction: 3'-phosphoadenosine 5'-phosphosulfate + an alcohol = adenosine 3',5'-bisphosphate + an alkyl sulfate. Also known as: estrogen sulfotransferase, steroid alcohol sulfotransferase, alcohol sulphotransferase activity, 3'-phosphoadenylyl-sulfate:alcohol sulfotransferase activity, 3-hydroxysteroid sulfotransferase activity, 3beta-hydroxy steroid sulfotransferase activity, 3beta-hydroxysteroid sulfotransferase activity, 5alpha-androstenol sulfotransferase activity, HST, alcohol/hydroxysteroid sulfotransferase activity, dehydroepiandrosterone sulfotransferase activity, delta5-3beta-hydroxysteroid sulfokinase activity, estrogen sulfokinase activity, hydroxysteroid sulfotransferase activity, steroid sulfokinase activity, sterol sulfokinase activity, sterol sulfotransferase activity Sources: EC:2.8.2.2 Subtypes: cholesterol sulfotransferase activity [GO:0051922] Relationships: is a type of sulfotransferase activity [GO:0008146]